cellular detoxification of copper ion [GO:1990880] (biological process) Relationships: is a type of detoxification of copper ion [GO:0010273]; is a type of cellular detoxification of metal ion [GO:0140961]; is part of cellular response to copper ion [GO:0071280] Definition: Any process that reduces or removes the toxicity of copper ions in a cell. These include transport of copper cations away from sensitive areas and to compartments or complexes whose purpose is sequestration. References: PMID:10369673